{
  "gene_name": "Secretoglobin family 1D member 1",
  "term_id": "UNKNOWN:0001",
  "gene": "UniProtKB:O95968",
  "term_label": "Unknown molecular function",
  "gene_symbol": "SCGB1D1"
}